{
  "gene_name": "Alpha-taxilin",
  "gene_symbol": "TXLNA",
  "gene": "UniProtKB:P40222",
  "term_id": "UNKNOWN:0001",
  "term_label": "Unknown molecular function"
}